{
  "gene": "UniProtKB:Q9QC07",
  "gene_symbol": "ERVK-18",
  "term_label": "Unknown cellular component",
  "gene_name": "Endogenous retrovirus group K member 18 Pol protein",
  "term_id": "UNKNOWN:0003"
}